{
  "term_label": "heat shock protein binding",
  "term_id": "GO:0031072",
  "gene_symbol": "TOMM34",
  "gene_name": "Mitochondrial import receptor subunit TOM34",
  "gene": "UniProtKB:Q15785"
}